{
  "term_label": "nucleus",
  "gene": "UniProtKB:Q6DCA0",
  "gene_symbol": "AMMECR1L",
  "term_id": "GO:0005634",
  "gene_name": "AMMECR1-like protein"
}